folate import into mitochondrion [GO:1904947] (biological process) References: PMID:15140890 Sources: GOC:BHF, GOC:TermGenie, GOC:rph, GO_REF:0000075 Definition: The process in which folic acid is transported from the cytosol into the mitochondrial matrix. Relationships: is a type of folate transmembrane transport [GO:0098838] Also known as: folic acid import into mitochondrion